{
  "gene_name": "von Willebrand factor A domain-containing protein 7",
  "term_label": "Unknown molecular function",
  "gene": "UniProtKB:Q9Y334",
  "gene_symbol": "VWA7",
  "term_id": "UNKNOWN:0001"
}